{
  "term_label": "calcium channel inhibitor activity",
  "gene_name": "Calcium uniporter regulatory subunit MCUb, mitochondrial",
  "gene": "UniProtKB:Q9NWR8",
  "gene_symbol": "MCUB",
  "term_id": "GO:0019855"
}